{
  "term_id": "GO:0006936",
  "term_label": "muscle contraction",
  "gene_name": "Myosin-8",
  "gene_symbol": "MYH8",
  "gene": "UniProtKB:P13535"
}